{
  "gene_symbol": "GALNT1",
  "gene_name": "Polypeptide N-acetylgalactosaminyltransferase 1",
  "term_label": "polypeptide N-acetylgalactosaminyltransferase activity",
  "term_id": "GO:0004653",
  "gene": "UniProtKB:Q10472"
}